{
  "gene_symbol": "UROD",
  "gene_name": "Uroporphyrinogen decarboxylase",
  "gene": "UniProtKB:P06132",
  "term_label": "cytosol",
  "term_id": "GO:0005829"
}